{
  "term_label": "cyclosporin A binding",
  "gene_name": "Peptidyl-prolyl cis-trans isomerase D",
  "term_id": "GO:0016018",
  "gene_symbol": "PPID",
  "gene": "UniProtKB:Q08752"
}